{
  "gene": "UniProtKB:Q9Y2V0",
  "gene_symbol": "CDIN1",
  "term_label": "cytoplasm",
  "gene_name": "CDAN1-interacting nuclease 1",
  "term_id": "GO:0005737"
}